transforming growth factor beta3 production [GO:0032907] (biological process) Relationships: is a type of transforming growth factor beta production [GO:0071604] Regulation: regulated by regulation of transforming growth factor beta3 production [GO:0032910]; RO_0002212 by negative regulation of transforming growth factor beta3 production [GO:0032913]; positively regulated by GO:0032916 Also known as: TGF-B3 production, TGFB3 production, transforming growth factor-beta3 production Definition: The appearance of transforming growth factor-beta3 due to biosynthesis or secretion following a cellular stimulus, resulting in an increase in its intracellular or extracellular levels. Sources: GOC:mah